{
  "gene_name": "Tubulointerstitial nephritis antigen",
  "gene_symbol": "TINAG",
  "term_label": "lysosome",
  "term_id": "GO:0005764",
  "gene": "UniProtKB:Q9UJW2"
}